{
  "gene": "UniProtKB:D6RF30",
  "gene_name": "Golgin subfamily A member 8K",
  "term_id": "UNKNOWN:0001",
  "gene_symbol": "GOLGA8K",
  "term_label": "Unknown molecular function"
}